{
  "gene": "UniProtKB:Q00610",
  "gene_name": "Clathrin heavy chain 1",
  "term_id": "GO:0032051",
  "term_label": "clathrin light chain binding",
  "gene_symbol": "CLTC"
}